{
  "gene_name": "Metallothionein-1A",
  "gene_symbol": "MT1A",
  "term_label": "metal ion binding",
  "term_id": "GO:0046872",
  "gene": "UniProtKB:P04731"
}